{
  "gene": "UniProtKB:Q03519",
  "term_id": "GO:0016020",
  "term_label": "membrane",
  "gene_symbol": "TAP2",
  "gene_name": "Antigen peptide transporter 2"
}